{
  "term_id": "UNKNOWN:0002",
  "term_label": "Unknown biological process",
  "gene": "UniProtKB:Q9NX76",
  "gene_name": "CKLF-like MARVEL transmembrane domain-containing protein 6",
  "gene_symbol": "CMTM6"
}